{
  "gene_name": "Guanine nucleotide-binding protein G(t) subunit alpha-2",
  "gene_symbol": "GNAT2",
  "term_id": "GO:0001664",
  "term_label": "G protein-coupled receptor binding",
  "gene": "UniProtKB:P19087"
}